Tapasin-ERp57 complex [GO:0061779] (CC) Definition: Subunit of the MHC class I peptide loading complex (GO:0042824) (=PLC) involved in the assembly of the heavy-chain-beta2-microglobulin dimers of the MHC class I molecules that fold with eight to ten residue peptides in the endoplasmic reticulum. Required for the inhibition of the reduction of the disulfide bonds of the heavy chains and the assembly and stabilization of the PLC, suggesting it may play a structural rather than a catalytic role. References: PMID:17603487 Sources: GOC:bhm, GOC:dph, Intact:EBI-11896237, Intact:EBI-9013963 Relationships: is a type of GO:0098796; is a type of endoplasmic reticulum protein-containing complex [GO:0140534]; is part of MHC class I peptide loading complex [GO:0042824]